{
  "gene": "UniProtKB:Q6PIL6",
  "gene_name": "Kv channel-interacting protein 4",
  "gene_symbol": "KCNIP4",
  "term_id": "GO:0009966",
  "term_label": "regulation of signal transduction"
}